{
  "gene": "UniProtKB:Q99700",
  "term_label": "stress granule assembly",
  "term_id": "GO:0034063",
  "gene_name": "Ataxin-2",
  "gene_symbol": "ATXN2"
}